{
  "term_id": "UNKNOWN:0003",
  "term_label": "Unknown cellular component",
  "gene": "UniProtKB:P53990",
  "gene_symbol": "IST1",
  "gene_name": "IST1 homolog"
}